histone H3K122 acetyltransferase activity [GO:0140908] (molecular function) Also known as: histone H3-K122 acetyltransferase activity, histone acetylase activity (H3-K122 specific), histone acetyltransferase activity (H3-K122 specific), histone lysine N-acetyltransferase activity (H3-K122 specific) References: PMID:23415232 Relationships: is a type of GO:0010484 Definition: Catalysis of the reaction: acetyl-CoA + histone H3 L-lysine (position 122) = CoA + histone H3 N6-acetyl-L-lysine (position 122). Note: Comment: Note that the residue position corresponds to the canonical human H3 histone (UniProtKB:P84243); this residue is conserved across all eukaryotes. Residue 1 is the first residue following removal of the initiating Methionine (Met). Note that each histone is encoded by multiple genes, and sequences may vary across different genes within an organism.